{
  "gene_symbol": "DIRAS1",
  "gene": "UniProtKB:O95057",
  "term_id": "GO:0003924",
  "gene_name": "GTP-binding protein Di-Ras1",
  "term_label": "GTPase activity"
}